{
  "gene": "UniProtKB:P54253",
  "gene_symbol": "ATXN1",
  "term_id": "GO:0000122",
  "term_label": "negative regulation of transcription by RNA polymerase II",
  "gene_name": "Ataxin-1"
}